UCC codon-amino acid adaptor activity [GO:0033406] (molecular function) Definition: A triplet codon-amino acid adaptor activity that recognizes a UCC codon. Sources: GOC:mah Also known as: TCC codon-amino acid adaptor activity, serine tRNA Note: Note that in the standard genetic code, TCC codes for serine. Relationships: is_a triplet codon-amino acid adaptor activity [GO:0030533]